flavin-containing compound catabolic process [GO:0042728] (biological process) Definition: The chemical reactions and pathways resulting in the breakdown of a flavin, any derivative of the dimethylisoalloxazine (7,8-dimethylbenzo[g]pteridine-2,4(3H,10H)-dione) skeleton, with a substituent on the 10 position. Sources: GOC:jl, GOC:mah Also known as: flavin-containing compound catabolic process breakdown, flavin-containing compound catabolic process degradation, flavin-containing compound catabolism, riboflavin and derivative catabolic process, riboflavin and derivative catabolism, vitamin B2 and derivative catabolic process, vitamin B2 and derivative catabolism Relationships: is a type of catabolic process [GO:0009056]; is a type of flavin-containing compound metabolic process [GO:0042726] Subtypes: riboflavin catabolic process [GO:0009232], FMN catabolic process [GO:0032363], flavin adenine dinucleotide catabolic process [GO:0072389]